{
  "term_id": "GO:0005737",
  "term_label": "cytoplasm",
  "gene_symbol": "DHX30",
  "gene_name": "ATP-dependent RNA helicase DHX30",
  "gene": "UniProtKB:Q7L2E3"
}